{
  "gene_symbol": "PDLIM1",
  "gene": "UniProtKB:O00151",
  "term_id": "GO:0030036",
  "term_label": "actin cytoskeleton organization",
  "gene_name": "PDZ and LIM domain protein 1"
}